{
  "gene_symbol": "FAM222A",
  "term_id": "UNKNOWN:0003",
  "gene": "UniProtKB:Q5U5X8",
  "gene_name": "Protein FAM222A",
  "term_label": "Unknown cellular component"
}